{
  "gene_symbol": "WRN",
  "gene_name": "Bifunctional 3'-5' exonuclease_ATP-dependent helicase WRN",
  "term_id": "GO:0006260",
  "gene": "UniProtKB:Q14191",
  "term_label": "DNA replication"
}